{
  "term_label": "positive regulation of transcription by RNA polymerase II",
  "term_id": "GO:0045944",
  "gene": "UniProtKB:Q86U70",
  "gene_symbol": "LDB1",
  "gene_name": "LIM domain-binding protein 1"
}